{
  "gene_name": "(3R)-3-hydroxyacyl-CoA dehydrogenase",
  "gene_symbol": "HSD17B8",
  "term_id": "GO:0004303",
  "term_label": "estradiol 17-beta-dehydrogenase [NAD(P)+] activity",
  "gene": "UniProtKB:Q92506"
}